peptidyl-glutaminase activity [GO:0050170] (molecular function) Relationships: is a type of GO:0016811 Definition: Catalysis of the reaction: alpha-N-peptidyl-L-glutamine + H2O = alpha-N-peptidyl-L-glutamate + NH3. Sources: EC:3.5.1.43, MetaCyc:PEPTIDYL-GLUTAMINASE-RXN Also known as: peptidoglutaminase I activity, peptideglutaminase activity, peptidoglutaminase activity, peptidyl-L-glutamine amidohydrolase activity